{
  "gene_name": "Uroplakin-3b-like protein 1",
  "gene_symbol": "UPK3BL1",
  "term_id": "GO:0016020",
  "gene": "UniProtKB:B0FP48",
  "term_label": "membrane"
}